{
  "term_id": "UNKNOWN:0002",
  "gene_symbol": "WDR37",
  "term_label": "Unknown biological process",
  "gene_name": "WD repeat-containing protein 37",
  "gene": "UniProtKB:Q9Y2I8"
}